{
  "term_label": "myosin II complex",
  "gene_name": "Myosin-4",
  "gene_symbol": "MYH4",
  "gene": "UniProtKB:Q9Y623",
  "term_id": "GO:0016460"
}